{
  "gene": "UniProtKB:Q9ULL1",
  "term_id": "GO:0005085",
  "gene_symbol": "PLEKHG1",
  "gene_name": "Pleckstrin homology domain-containing family G member 1",
  "term_label": "guanyl-nucleotide exchange factor activity"
}